{
  "gene_name": "Testis-expressed protein 36",
  "term_label": "Unknown biological process",
  "gene": "UniProtKB:Q5VZQ5",
  "gene_symbol": "TEX36",
  "term_id": "UNKNOWN:0002"
}